{
  "term_id": "GO:0061665",
  "term_label": "SUMO ligase activity",
  "gene_symbol": "PIAS2",
  "gene_name": "E3 SUMO-protein ligase PIAS2",
  "gene": "UniProtKB:O75928"
}